{
  "gene": "UniProtKB:A0A8V8TMC4",
  "gene_symbol": "CCNYL1B",
  "term_id": "GO:0061575",
  "gene_name": "Cyclin N-terminal domain-containing protein",
  "term_label": "cyclin-dependent protein serine/threonine kinase activator activity"
}